{
  "term_label": "nucleus",
  "term_id": "GO:0005634",
  "gene": "UniProtKB:O60248",
  "gene_name": "Protein SOX-15",
  "gene_symbol": "SOX15"
}